symbiont-mediated suppression of host anti-inflammatory cytokine signaling [GO:0141174] (biological process) References: PMID:19168731, PMID:29720526, PMID:32754056 Relationships: is a type of symbiont-mediated perturbation of host receptor-mediated signal transduction [GO:0075109] Also known as: negative regulation by symbiont of host anti-inflammatory cytokine production, suppression by symbiont of host anti-inflammatory cytokine production, symbiont-mediated degradation of host anti-inflammatory cytokine, suppression by symbiont of host anti-inflammatory cytokine secretion, symbiont-mediated sequestering of host anti-inflammatory cytokine, symbiont-mediated suppression of host anti-inflammatory cytokine production Definition: A process by which a symbiont inhibits or disrupts anti-inflammatory cytokine signaling in the host organism, either by disruption of production, sequesteration, or destruction of at least one component of the signaling pathway.  Anti-inflammatory cytokines include: interleukin (IL)-1, IL-4, IL-6, IL-10, IL-11, and IL-13. The host is defined as the larger of the organisms involved in a symbiotic interaction.